{
  "term_label": "regulation of cell cycle phase transition",
  "term_id": "GO:1901987",
  "gene_name": "Cyclin-dependent kinase 18",
  "gene": "UniProtKB:Q07002",
  "gene_symbol": "CDK18"
}